positive regulation of interleukin-26 production [GO:0032750] (biological process) Relationships: is a type of positive regulation of cytokine production [GO:0001819]; is_a regulation of interleukin-26 production [GO:0032670]; positively regulates GO:0032630 Definition: Any process that activates or increases the frequency, rate, or extent of interleukin-26 production. Sources: GOC:mah Also known as: positive regulation of IL-26 production, up regulation of interleukin-26 production, up-regulation of interleukin-26 production, upregulation of interleukin-26 production, activation of interleukin-26 production, positive regulation of interleukin-26 biosynthetic process, stimulation of interleukin-26 production